{
  "gene_name": "Forkhead box protein Q1",
  "term_id": "UNKNOWN:0003",
  "term_label": "Unknown cellular component",
  "gene": "UniProtKB:Q9C009",
  "gene_symbol": "FOXQ1"
}